{
  "gene": "UniProtKB:Q9UKS6",
  "term_id": "GO:0097320",
  "gene_symbol": "PACSIN3",
  "gene_name": "Protein kinase C and casein kinase substrate in neurons protein 3",
  "term_label": "plasma membrane tubulation"
}